{
  "term_label": "mRNA binding",
  "term_id": "GO:0003729",
  "gene": "UniProtKB:P08621",
  "gene_symbol": "SNRNP70",
  "gene_name": "U1 small nuclear ribonucleoprotein 70 kDa"
}